microtubule nucleation [GO:0007020] (biological process) Subtypes: microtubule nucleation by microtubule organizing center [GO:0051418], GO:0090221, chromatin-templated microtubule nucleation [GO:0090223] References: PMID:12517712 Sources: GOC:go_curators, ISBN:0815316194 Regulation: regulated by regulation of microtubule nucleation [GO:0010968]; positively regulated by positive regulation of microtubule nucleation [GO:0090063]; RO_0002212 by GO:1905833 Definition: The process in which tubulin alpha-beta heterodimers begin aggregation to form an oligomeric tubulin structure (a microtubule seed). Microtubule nucleation is the initiating step in the formation of a microtubule in the absence of any existing microtubules ('de novo' microtubule formation). Relationships: is a type of microtubule cytoskeleton organization [GO:0000226]; is part of GO:0046785